thioether S-methyltransferase activity [GO:0004790] (molecular function) Definition: Catalysis of the reaction: S-adenosyl-L-methionine(1+) + dimethyl sulfide = S-adenosyl-L-homocysteine + trimethylsulfonium. Sources: EC:2.1.1.96, RHEA:19613 Relationships: is a type of S-methyltransferase activity [GO:0008172]; is a type of GO:0008757 Also known as: S-adenosyl-L-methionine:dimethyl-sulfide S-methyltransferase activity, S-adenosyl-L-methionine:thioether S-methyltransferase activity, thioether methyltransferase activity